{
  "gene_name": "Heparan sulfate glucosamine 3-O-sulfotransferase 3A1",
  "term_id": "UNKNOWN:0002",
  "gene": "UniProtKB:Q9Y663",
  "gene_symbol": "HS3ST3A1",
  "term_label": "Unknown biological process"
}